oxidoreductase activity, acting on diphenols and related substances as donors, oxygen as acceptor [GO:0016682] (molecular function) Sources: GOC:jl Definition: Catalysis of an oxidation-reduction (redox) reaction in which a diphenol, or related compound, acts as a hydrogen or electron donor and reduces oxygen. Subtypes: catechol oxidase activity [GO:0004097], GO:0008447, alternative oxidase activity [GO:0009916], 3-hydroxyanthranilate oxidase activity [GO:0047561], o-aminophenol oxidase activity [GO:0050149], rifamycin-B oxidase activity [GO:0050264], hydroquinone:oxygen oxidoreductase activity [GO:0052716], GO:0102721 Also known as: laccase activity Relationships: is a type of GO:0016679